somatic hypermutation of immunoglobulin genes involved in immune response [GO:0002205] (biological process) References: PMID:11205333, PMID:14991701 Sources: GOC:add, ISBN:0781735149 Also known as: somatic hypermutation of antibody genes during immune response, somatic hypermutation of immunoglobulin genes during immune response Definition: Mutations occurring somatically that result in amino acid changes in the rearranged V regions of immunoglobulins following the induction of and contributing to an immune response. Relationships: is_a GO:0002208; is a type of GO:0016446; is part of B cell affinity maturation [GO:0002344]